{
  "gene_name": "All trans-polyprenyl-diphosphate synthase PDSS2",
  "term_label": "polyprenyl diphosphate synthase complex",
  "gene_symbol": "PDSS2",
  "term_id": "GO:0032476",
  "gene": "UniProtKB:Q86YH6"
}